{
  "gene_symbol": "ADCY5",
  "gene": "UniProtKB:O95622",
  "gene_name": "Adenylate cyclase type 5",
  "term_label": "cAMP biosynthetic process",
  "term_id": "GO:0006171"
}